{
  "term_label": "Unknown molecular function",
  "gene": "UniProtKB:Q9NXV6",
  "gene_name": "CDKN2A-interacting protein",
  "gene_symbol": "CDKN2AIP",
  "term_id": "UNKNOWN:0001"
}